iron-sulfur-molybdenum cofactor biosynthetic process [GO:1901288] (biological process) Definition: The chemical reactions and pathways resulting in the formation of iron-sulfur-molybdenum cofactor. Also known as: FeMo-co anabolism, FeMo-co biosynthesis, FeMo-co biosynthetic process, FeMo-co formation, FeMo-co synthesis, iron-molybdenum cofactor anabolism, iron-molybdenum cofactor biosynthesis, iron-molybdenum cofactor biosynthetic process, iron-molybdenum cofactor formation, iron-molybdenum cofactor synthesis, iron-sulfur-molybdenum cofactor anabolism, iron-sulfur-molybdenum cofactor biosynthesis, iron-sulfur-molybdenum cofactor formation, iron-sulfur-molybdenum cofactor synthesis Sources: GOC:TermGenie, GOC:yaf, UniPathway:UPA00782 Relationships: is a type of biosynthetic process [GO:0009058]; is a type of iron-sulfur-molybdenum cofactor metabolic process [GO:1901286]